{
  "term_id": "GO:0003677",
  "gene_name": "Chromodomain-helicase-DNA-binding protein 4",
  "term_label": "DNA binding",
  "gene_symbol": "CHD4",
  "gene": "UniProtKB:Q14839"
}